{
  "gene_symbol": "CHRNG",
  "term_label": "synapse",
  "gene_name": "Acetylcholine receptor subunit gamma",
  "gene": "UniProtKB:P07510",
  "term_id": "GO:0045202"
}